{
  "gene_name": "Calcium and integrin-binding family member 4",
  "gene_symbol": "CIB4",
  "term_label": "magnesium ion binding",
  "gene": "UniProtKB:A0PJX0",
  "term_id": "GO:0000287"
}